regulation of cell cycle switching, mitotic to meiotic cell cycle [GO:0110044] (biological process) Subtypes: negative regulation of cell cycle switching, mitotic to meiotic cell cycle [GO:0110045], GO:0140648 Also known as: sexual differentiation Relationships: is_a regulation of mitotic cell cycle [GO:0007346]; is a type of regulation of cell cycle process [GO:0010564]; is_a regulation of meiotic cell cycle [GO:0051445]; regulates cell cycle switching, mitotic to meiotic cell cycle [GO:0051728] Definition: Any process that modulates the frequency, rate, or extent of mitotic to meiotic cell cycle switching, the process in which a cell switches cell cycle mode from mitotic to meiotic division. References: PMID:17674143 Sources: GOC:al